regulation of cytolysis [GO:0042268] (biological process) Definition: Any process that modulates the frequency, rate or extent of the rupture of cell membranes and the loss of cytoplasm. Sources: GOC:jl, GOC:mtg_apoptosis Relationships: is a type of regulation of cellular process [GO:0050794]; regulates cytolysis [GO:0019835] Subtypes: negative regulation of cytolysis [GO:0045918], positive regulation of cytolysis [GO:0045919]